Golgi ribbon formation [GO:0090161] (biological process) Sources: GOC:ascb_2009, GOC:dph, GOC:tb Definition: The formation of a continuous ribbon of interconnected Golgi stacks of flat cisternae. Subtypes: GO:0090164 Relationships: is a type of Golgi organization [GO:0007030]